{
  "gene_name": "F-box only protein 3",
  "term_label": "cytoplasm",
  "term_id": "GO:0005737",
  "gene": "UniProtKB:Q9UK99",
  "gene_symbol": "FBXO3"
}